{
  "term_label": "focal adhesion",
  "gene_name": "Vinculin",
  "gene_symbol": "VCL",
  "gene": "UniProtKB:P18206",
  "term_id": "GO:0005925"
}